{
  "term_label": "hair follicle development",
  "gene_symbol": "LOC112267897",
  "term_id": "GO:0001942",
  "gene_name": "Uncharacterized protein",
  "gene": "UniProtKB:A0A3B3IRQ3"
}